{
  "gene_symbol": "TMEM104",
  "term_label": "Unknown biological process",
  "gene": "UniProtKB:Q8NE00",
  "term_id": "UNKNOWN:0002",
  "gene_name": "Transmembrane protein 104"
}